{
  "term_id": "GO:0008250",
  "gene_symbol": "DDOST",
  "term_label": "oligosaccharyltransferase complex",
  "gene": "UniProtKB:P39656",
  "gene_name": "Dolichyl-diphosphooligosaccharide--protein glycosyltransferase 48 kDa subunit"
}